{
  "gene": "UniProtKB:Q13641",
  "term_id": "GO:0090090",
  "gene_symbol": "TPBG",
  "term_label": "negative regulation of canonical Wnt signaling pathway",
  "gene_name": "Trophoblast glycoprotein"
}